{
  "gene_symbol": "OR52N2",
  "gene": "UniProtKB:Q8NGI0",
  "term_id": "UNKNOWN:0002",
  "gene_name": "Olfactory receptor 52N2",
  "term_label": "Unknown biological process"
}